{
  "term_id": "GO:0008020",
  "gene": "UniProtKB:Q6U736",
  "gene_symbol": "OPN5",
  "term_label": "G protein-coupled photoreceptor activity",
  "gene_name": "Opsin-5"
}